{
  "gene": "UniProtKB:O75818",
  "term_label": "endonucleolytic cleavage in ITS1 to separate SSU-rRNA from 5.8S rRNA and LSU-rRNA from tricistronic rRNA transcript (SSU-rRNA, 5.8S rRNA, LSU-rRNA)",
  "gene_symbol": "RPP40",
  "gene_name": "Ribonuclease P protein subunit p40",
  "term_id": "GO:0000447"
}